{
  "term_id": "GO:0015645",
  "gene": "UniProtKB:Q08AH3",
  "term_label": "fatty acid ligase activity",
  "gene_name": "Acyl-coenzyme A synthetase ACSM2A, mitochondrial",
  "gene_symbol": "ACSM2A"
}